{
  "term_label": "gamma-aminobutyric acid signaling pathway",
  "gene": "UniProtKB:P31644",
  "gene_symbol": "GABRA5",
  "term_id": "GO:0007214",
  "gene_name": "Gamma-aminobutyric acid receptor subunit alpha-5"
}